negative regulation of fumigaclavine C biosynthetic process [GO:1900838] (biological process) Definition: Any process that stops, prevents or reduces the frequency, rate or extent of fumigaclavine C biosynthetic process. Sources: GOC:TermGenie, GOC:di Also known as: inhibition of fumigaclavine C biosynthetic process Relationships: is a type of negative regulation of ergot alkaloid biosynthetic process [GO:1900823]; is a type of regulation of fumigaclavine C biosynthetic process [GO:1900837]; negatively regulates fumigaclavine C biosynthetic process [GO:1900809]